{
  "gene_name": "Polyphosphoinositide phosphatase",
  "gene_symbol": "FIG4",
  "gene": "UniProtKB:Q92562",
  "term_id": "GO:0043813",
  "term_label": "phosphatidylinositol-3,5-bisphosphate 5-phosphatase activity"
}